{
  "gene_name": "DnaJ homolog subfamily A member 4",
  "term_id": "GO:0051082",
  "gene_symbol": "DNAJA4",
  "term_label": "unfolded protein binding",
  "gene": "UniProtKB:Q8WW22"
}